{
  "term_id": "GO:0003723",
  "gene_symbol": "RPL7L1",
  "gene": "UniProtKB:Q6DKI1",
  "term_label": "RNA binding",
  "gene_name": "Ribosomal protein uL30-like"
}